{
  "term_label": "cytoskeleton",
  "gene": "UniProtKB:Q9NR20",
  "gene_name": "Dual specificity tyrosine-phosphorylation-regulated kinase 4",
  "term_id": "GO:0005856",
  "gene_symbol": "DYRK4"
}